{
  "gene": "UniProtKB:P01906",
  "term_id": "GO:0019886",
  "gene_name": "HLA class II histocompatibility antigen, DQ alpha 2 chain",
  "term_label": "antigen processing and presentation of exogenous peptide antigen via MHC class II",
  "gene_symbol": "HLA-DQA2"
}